{
  "term_label": "lysosome",
  "term_id": "GO:0005764",
  "gene_symbol": "CLN3",
  "gene": "UniProtKB:Q13286",
  "gene_name": "Battenin"
}